{
  "term_label": "cellular response to leucine starvation",
  "gene_name": "Sestrin-1",
  "gene": "UniProtKB:Q9Y6P5",
  "term_id": "GO:1990253",
  "gene_symbol": "SESN1"
}